{
  "term_label": "regulation of alternative mRNA splicing, via spliceosome",
  "gene": "UniProtKB:Q9UHX1",
  "gene_symbol": "PUF60",
  "term_id": "GO:0000381",
  "gene_name": "Poly(U)-binding-splicing factor PUF60"
}